{
  "term_label": "Unknown cellular component",
  "term_id": "UNKNOWN:0003",
  "gene": "UniProtKB:Q6X4T0",
  "gene_name": "Uncharacterized protein C12orf54",
  "gene_symbol": "C12orf54"
}